{
  "term_id": "GO:0005829",
  "gene": "UniProtKB:P32320",
  "gene_name": "Cytidine deaminase",
  "gene_symbol": "CDA",
  "term_label": "cytosol"
}